autolysosome lumen [GO:0120282] (cellular component) References: PMID:17182262, PMID:24657946, PMID:26382870, PMID:32047650 Sources: GOC:krc, GOC:nhn Definition: The volume that is enclosed within the autolysosome single-membrane. Relationships: is a type of GO:0005775; is part of autolysosome [GO:0044754]